{
  "gene_name": "Protein-arginine deiminase type-1",
  "gene": "UniProtKB:Q9ULC6",
  "gene_symbol": "PADI1",
  "term_id": "UNKNOWN:0002",
  "term_label": "Unknown biological process"
}